{
  "term_label": "MLL1 complex",
  "gene_name": "MAX gene-associated protein",
  "gene": "UniProtKB:Q8IWI9",
  "gene_symbol": "MGA",
  "term_id": "GO:0071339"
}